{
  "term_label": "neurogenesis",
  "gene_name": "WD repeat-containing protein 62",
  "gene_symbol": "WDR62",
  "gene": "UniProtKB:O43379",
  "term_id": "GO:0022008"
}